{
  "term_label": "U2 snRNP",
  "gene_name": "Small nuclear ribonucleoprotein E",
  "gene_symbol": "SNRPE",
  "gene": "UniProtKB:P62304",
  "term_id": "GO:0005686"
}